{
  "term_id": "UNKNOWN:0002",
  "gene_name": "HCG2039779 (Fragment)",
  "term_label": "Unknown biological process",
  "gene": "UniProtKB:A0N4Z8",
  "gene_symbol": "TRAJ9"
}